{
  "gene": "UniProtKB:Q14031",
  "term_id": "GO:0031012",
  "gene_symbol": "COL4A6",
  "gene_name": "Collagen alpha-6(IV) chain",
  "term_label": "extracellular matrix"
}